{
  "gene_symbol": "ZNF439",
  "gene": "UniProtKB:Q8NDP4",
  "term_label": "regulation of transcription by RNA polymerase II",
  "term_id": "GO:0006357",
  "gene_name": "Zinc finger protein 439"
}